{
  "term_label": "unfolded protein binding",
  "gene": "UniProtKB:P50991",
  "gene_name": "T-complex protein 1 subunit delta",
  "term_id": "GO:0051082",
  "gene_symbol": "CCT4"
}